morphine receptor activity [GO:0038047] (molecular function) Definition: Combining with morphine (17-methyl-7,8-didehydro-4,5alpha-epoxymorphinan-3,6alpha-diol), and transmitting the signal across the membrane by activating an associated G-protein. Also known as: mu-opioid receptor activity Sources: GOC:bf Relationships: is a type of GO:0004985; is part of cellular response to morphine [GO:0071315]